{
  "gene_name": "Nucleoside diphosphate-linked moiety X motif 6",
  "term_label": "Unknown cellular component",
  "gene_symbol": "NUDT6",
  "gene": "UniProtKB:P53370",
  "term_id": "UNKNOWN:0003"
}